{
  "term_label": "regulation of transcription by RNA polymerase II",
  "gene": "UniProtKB:Q8N7K0",
  "gene_symbol": "ZNF433",
  "gene_name": "Zinc finger protein 433",
  "term_id": "GO:0006357"
}